{
  "term_label": "high-density lipoprotein particle binding",
  "gene_symbol": "APOA2",
  "gene": "UniProtKB:P02652",
  "term_id": "GO:0008035",
  "gene_name": "Apolipoprotein A-II"
}